serotonin biosynthetic process from tryptophan [GO:0006587] (BP) Sources: GOC:jl, ISBN:0198506732 Also known as: serotonin anabolism from tryptophan, serotonin formation from tryptophan, serotonin synthesis from tryptophan Definition: The chemical reactions and pathways resulting in the formation from tryptophan of serotonin (5-hydroxytryptamine), a monoamine neurotransmitter occurring in the peripheral and central nervous systems, also having hormonal properties. Relationships: is a type of GO:0009072; is a type of GO:0042427; is a type of alpha-amino acid metabolic process [GO:1901605]